{
  "term_label": "Unknown biological process",
  "gene_symbol": "PNMA5",
  "gene": "UniProtKB:Q96PV4",
  "gene_name": "Paraneoplastic antigen-like protein 5",
  "term_id": "UNKNOWN:0002"
}